{
  "gene_name": "Paralemmin-2",
  "term_label": "Unknown biological process",
  "term_id": "UNKNOWN:0002",
  "gene": "UniProtKB:Q8IXS6",
  "gene_symbol": "PALM2"
}